indoleacetic acid biosynthetic process [GO:0009684] (biological process) Also known as: IAA biosynthetic process, indole acetic acid biosynthesis, indole acetic acid biosynthetic process, indole-3-acetate biosynthesis, indole-3-acetate biosynthetic process, indole-acetic acid biosynthesis, indoleacetic acid anabolism, indoleacetic acid biosynthesis, indoleacetic acid formation, indoleacetic acid synthesis, indole-acetic acid biosynthetic process Relationships: is a type of auxin biosynthetic process [GO:0009851]; is a type of indole-containing compound biosynthetic process [GO:0042435]; is_a monocarboxylic acid biosynthetic process [GO:0072330] Subtypes: indoleacetic acid biosynthetic process via tryptophan [GO:0009848], tryptophan-independent indoleacetic acid biosynthetic process [GO:0009849] Sources: ISBN:0387969845 Definition: The chemical reactions and pathways resulting in the formation of indole-3-acetic acid, a compound which functions as a growth regulator in plants.